{
  "gene_symbol": "PXMP2",
  "term_label": "peroxisomal membrane",
  "term_id": "GO:0005778",
  "gene": "UniProtKB:Q9NR77",
  "gene_name": "Peroxisomal membrane protein 2"
}